{
  "gene_symbol": "KMT2D",
  "term_label": "MLL3/4 complex",
  "term_id": "GO:0044666",
  "gene_name": "Histone-lysine N-methyltransferase 2D",
  "gene": "UniProtKB:O14686"
}